{
  "term_id": "GO:0005634",
  "gene": "UniProtKB:P57682",
  "gene_name": "Krueppel-like factor 3",
  "gene_symbol": "KLF3",
  "term_label": "nucleus"
}